{
  "gene": "UniProtKB:Q14573",
  "gene_name": "Inositol 1,4,5-trisphosphate receptor type 3",
  "term_id": "GO:0051209",
  "gene_symbol": "ITPR3",
  "term_label": "release of sequestered calcium ion into cytosol"
}